meiosis I cell cycle phase [GO:0098764] (biological process) Note: Note that this term should not be used for direct annotation. If you are trying to make an annotation to x phase, it is likely that the correct annotation is 'regulation of x/y phase transition' or to a process which occurs during the reported phase (i.e mitotic DNA replication for mitotic S-phase). To capture the phase when a specific location or process is observed, the phase term can be used in an annotation extension (PMID:24885854) applied to a cellular component term (with the relation exists_during) or a biological process term (with the relation happens_during). Relationships: is a type of meiotic cell cycle phase [GO:0098762] Definition: A meiotic cell cycle phase prior to a during which some part of meiosis I nuclear division or the proceeding cytokinesis occurs. Sources: GOC:dos Subtypes: leptotene [GO:0000237], zygotene [GO:0000238], GO:0000239, diplotene [GO:0000240], diakinesis [GO:0000241], meiotic prophase I [GO:0007128], meiotic metaphase I [GO:0007132], meiotic anaphase I [GO:0007133], meiotic telophase I [GO:0007134], meiotic prometaphase I [GO:0098768]